acetylputrescine deacetylase activity [GO:0047609] (molecular function) Definition: Catalysis of the reaction: N-acetylputrescine + H2O = acetate + putrescine. Sources: EC:3.5.1.62, RHEA:23412 Also known as: N-acetylputrescine acetylhydrolase activity Relationships: is a type of hydrolase activity, acting on carbon-nitrogen (but not peptide) bonds, in linear amides [GO:0016811]; is a type of deacetylase activity [GO:0019213]